{
  "term_id": "GO:0004198",
  "gene_name": "Calpain-9",
  "term_label": "calcium-dependent cysteine-type endopeptidase activity",
  "gene": "UniProtKB:O14815",
  "gene_symbol": "CAPN9"
}